{
  "gene": "UniProtKB:Q8IVU9",
  "term_id": "UNKNOWN:0001",
  "term_label": "Unknown molecular function",
  "gene_name": "Ciliary-associated calcium-binding coiled-coil protein 1",
  "gene_symbol": "CABCOCO1"
}